{
  "gene_symbol": "PRIM2",
  "term_id": "GO:0006269",
  "gene": "UniProtKB:P49643",
  "term_label": "DNA replication, synthesis of primer",
  "gene_name": "DNA primase large subunit"
}